{
  "gene": "UniProtKB:Q8NHW3",
  "gene_name": "Transcription factor MafA",
  "term_id": "GO:0030073",
  "term_label": "insulin secretion",
  "gene_symbol": "MAFA"
}